{
  "term_id": "GO:0003714",
  "gene_symbol": "AJUBA",
  "term_label": "transcription corepressor activity",
  "gene_name": "LIM domain-containing protein ajuba",
  "gene": "UniProtKB:Q96IF1"
}